regulation of stomatal complex development [GO:2000038] (biological process) Definition: Any process that modulates the frequency, rate or extent of stomatal complex development. Relationships: is a type of regulation of post-embryonic development [GO:0048580]; regulates stomatal complex development [GO:0010374] Sources: GOC:obol Subtypes: negative regulation of stomatal complex development [GO:2000122], positive regulation of stomatal complex development [GO:2000123]